{
  "term_id": "UNKNOWN:0001",
  "term_label": "Unknown molecular function",
  "gene_name": "Huntingtin",
  "gene_symbol": "HTT",
  "gene": "UniProtKB:P42858"
}